{
  "gene": "UniProtKB:Q8NHS4",
  "gene_name": "Clathrin heavy chain linker domain-containing protein 1",
  "term_id": "UNKNOWN:0002",
  "gene_symbol": "CLHC1",
  "term_label": "Unknown biological process"
}